regulation of purine nucleotide metabolic process [GO:1900542] (biological process) Relationships: is a type of regulation of nucleotide metabolic process [GO:0006140]; regulates purine nucleotide metabolic process [GO:0006163] Subtypes: regulation of purine nucleotide catabolic process [GO:0033121], regulation of purine nucleotide biosynthetic process [GO:1900371], negative regulation of purine nucleotide metabolic process [GO:1900543], positive regulation of purine nucleotide metabolic process [GO:1900544], regulation of NADP metabolic process [GO:1902031], regulation of NAD metabolic process [GO:1902688], regulation of ATP metabolic process [GO:1903578] Sources: GOC:TermGenie Definition: Any process that modulates the frequency, rate or extent of purine nucleotide metabolic process. Also known as: regulation of purine nucleotide metabolism, regulation of purine metabolic process, regulation of purine metabolism